{
  "term_label": "single-stranded DNA binding",
  "gene_symbol": "MCM9",
  "gene": "UniProtKB:Q9NXL9",
  "gene_name": "DNA helicase MCM9",
  "term_id": "GO:0003697"
}